{
  "gene_name": "BMP_retinoic acid-inducible neural-specific protein 2",
  "gene": "UniProtKB:Q9C0B6",
  "term_id": "GO:0030425",
  "gene_symbol": "BRINP2",
  "term_label": "dendrite"
}